{
  "gene_symbol": "ATG9A",
  "gene_name": "Autophagy-related protein 9A",
  "term_label": "reticulophagy",
  "gene": "UniProtKB:Q7Z3C6",
  "term_id": "GO:0061709"
}